{
  "gene": "UniProtKB:B4DJY2",
  "gene_name": "Transmembrane protein 233",
  "term_id": "UNKNOWN:0001",
  "term_label": "Unknown molecular function",
  "gene_symbol": "TMEM233"
}